{
  "term_label": "Unknown cellular component",
  "term_id": "UNKNOWN:0003",
  "gene": "UniProtKB:A0A286YEX9",
  "gene_symbol": "SCYGR10",
  "gene_name": "Small cysteine and glycine repeat-containing protein 10"
}